zinc:bicarbonate:selenite symporter activity [GO:0140413] (molecular function) Relationships: is a type of GO:0140412 Also known as: zinc:hydrogencarbonate:selenate symporter activity References: PMID:27166256 Definition: Enables the transfer of a solute or solutes from one side of a membrane to the other according to the reaction: zinc(out) + HCO3-(out) + HO3Se-(out) = zinc(in) + HCO3-(in) + HO3Se-(out).